{
  "term_id": "GO:0052689",
  "term_label": "carboxylic ester hydrolase activity",
  "gene_name": "Protein ABHD11",
  "gene": "UniProtKB:Q8NFV4",
  "gene_symbol": "ABHD11"
}